positive regulation of viral transcription [GO:0050434] (biological process) Definition: Any process that activates or increases the frequency, rate or extent of viral transcription. Sources: GOC:ai Also known as: up regulation of viral transcription, up-regulation of viral transcription, upregulation of viral transcription, activation of viral transcription, stimulation of viral transcription Relationships: is a type of regulation of viral transcription [GO:0046782]; is_a positive regulation of viral process [GO:0048524]; positively regulates viral transcription [GO:0019083]